{
  "gene": "UniProtKB:Q9UGI8",
  "term_label": "Unknown biological process",
  "gene_name": "Testin",
  "term_id": "UNKNOWN:0002",
  "gene_symbol": "TES"
}